{
  "gene_symbol": "SYT14",
  "term_id": "UNKNOWN:0002",
  "gene": "UniProtKB:Q8NB59",
  "gene_name": "Synaptotagmin-14",
  "term_label": "Unknown biological process"
}